luteolin-7-O-diglucuronide 4'-O-glucuronosyltransferase activity [GO:0047247] (molecular function) Definition: Catalysis of the reaction: luteolin 7-O-[(beta-D-glucosiduronate)-(1->2)-(beta-D-glucosiduronate)] + UDP-alpha-D-glucuronate = H+ + luteolin 7-O-[(beta-D-glucosiduronate)-(1->2)-(beta-D-glucosiduronate)] 4'-O-beta-D-glucosiduronate + UDP. Sources: EC:2.4.1.191, RHEA:22116 Also known as: LDT, UDP-glucuronate:luteolin 7-O-diglucuronide-glucuronosyltransferase activity, UDP-glucuronate:luteolin-7-O-beta-D-diglucuronide 4'-O-glucuronosyltransferase activity, UDPglucuronate:luteolin 7-O-diglucuronide-4'-O-glucuronosyl-transferase activity, UDPglucuronate:luteolin-7-O-beta-D-diglucuronide 4'-O-glucuronosyltransferase activity, uridine diphosphoglucuronate-luteolin 7-O-diglucuronide glucuronosyltransferase activity Relationships: is a type of glucuronosyltransferase activity [GO:0015020]